{
  "gene_name": "Urokinase plasminogen activator surface receptor",
  "term_id": "UNKNOWN:0001",
  "gene_symbol": "PLAUR",
  "term_label": "Unknown molecular function",
  "gene": "UniProtKB:Q03405"
}